{
  "gene": "UniProtKB:Q8NBJ4",
  "term_label": "Golgi apparatus",
  "gene_symbol": "GOLM1",
  "term_id": "GO:0005794",
  "gene_name": "Golgi membrane protein 1"
}